positive regulation of antipodal cell differentiation [GO:0045690] (biological process) Relationships: is a type of GO:0045597; is a type of regulation of antipodal cell differentiation [GO:0045688]; is_a positive regulation of multicellular organismal process [GO:0051240]; positively regulates antipodal cell differentiation [GO:0009557] Definition: Any process that activates or increases the frequency, rate or extent of antipodal cell differentiation. Sources: GOC:go_curators, GOC:mtg_plant Also known as: up regulation of antipodal cell differentiation, up-regulation of antipodal cell differentiation, upregulation of antipodal cell differentiation, activation of antipodal cell differentiation, stimulation of antipodal cell differentiation